ADP-ribose diphosphatase activity [GO:0047631] (molecular function) Definition: Catalysis of the reaction: ADP-ribose + H2O = AMP + D-ribose 5-phosphate. Also known as: ADP-ribose phosphohydrolase activity, ADP-ribose pyrophosphatase activity, ADPR-PPase activity, adenosine diphosphoribose pyrophosphatase activity, ADP-ribose ribophosphohydrolase activity, ADPribose diphosphatase activity, ADPribose pyrophosphatase activity Relationships: is a type of pyrophosphatase activity [GO:0016462] Sources: EC:3.6.1.13